{
  "gene_symbol": "CAPN2",
  "gene_name": "Calpain-2 catalytic subunit",
  "term_label": "proteolysis",
  "gene": "UniProtKB:P17655",
  "term_id": "GO:0006508"
}